{
  "term_id": "GO:0140374",
  "term_label": "antiviral innate immune response",
  "gene": "UniProtKB:Q13325",
  "gene_symbol": "IFIT5",
  "gene_name": "Interferon-induced protein with tetratricopeptide repeats 5"
}